{
  "gene_symbol": "COMTD1",
  "term_id": "GO:0008757",
  "term_label": "S-adenosylmethionine-dependent methyltransferase activity",
  "gene": "UniProtKB:Q86VU5",
  "gene_name": "Catechol O-methyltransferase domain-containing protein 1"
}